cellular response to fluid shear stress [GO:0071498] (biological process) Definition: Any process that results in a change in state or activity of a cell (in terms of movement, secretion, enzyme production, gene expression, etc.) as a result of a fluid shear stress stimulus. Fluid shear stress is the force acting on an object in a system where the fluid is moving across a solid surface. Sources: GOC:mah Relationships: is a type of cellular response to stress [GO:0033554]; is a type of GO:0034405 Subtypes: GO:0071499, vascular endothelial cell response to fluid shear stress [GO:0097699], GO:0097703, cellular response to oscillatory fluid shear stress [GO:0097704]